{
  "gene_name": "Tryptophan--tRNA ligase, mitochondrial",
  "gene_symbol": "WARS2",
  "gene": "UniProtKB:Q9UGM6",
  "term_label": "mitochondrial matrix",
  "term_id": "GO:0005759"
}